poly-glutamine tract binding [GO:0008267] (molecular function) Sources: GOC:mah Relationships: is a type of protein binding [GO:0005515] Definition: Binding to a polyglutamine tract, i.e. a series of consecutive glutamine residues, in a protein.